alphaV-beta3 integrin-gelsolin complex [GO:0071096] (cellular component) Relationships: is a type of plasma membrane protein complex [GO:0098797] References: PMID:11577104 Also known as: ITGAV-ITGB3-Gsn complex Definition: A protein complex that consists of an alphaV-beta3 integrin complex bound to gelsolin.